{
  "gene": "UniProtKB:Q5TID7",
  "term_id": "UNKNOWN:0002",
  "gene_symbol": "CCDC181",
  "gene_name": "Coiled-coil domain-containing protein 181",
  "term_label": "Unknown biological process"
}